{
  "term_id": "GO:0031012",
  "gene": "UniProtKB:Q15582",
  "term_label": "extracellular matrix",
  "gene_name": "Transforming growth factor-beta-induced protein ig-h3",
  "gene_symbol": "TGFBI"
}